cerebellar cortex formation [GO:0021697] (biological process) Sources: GOC:cls, GOC:dgh, GOC:dph, GOC:jid, GO_REF:0000021 Relationships: is a type of GO:0048646; is part of cerebellar cortex morphogenesis [GO:0021696] Definition: The process that gives rise to the cerebellar cortex. This process pertains to the initial formation of a structure from unspecified parts. The cerebellar cortex is a thin mantle of gray matter that covers the surface of each cerebral hemisphere. It has a characteristic morphology with convolutions (gyri) and crevices (sulci) that have specific functions. Six layers of nerve cells and the nerve pathways that connect them comprise the cerebellar cortex. Together, these regions are responsible for the processes of conscious thought, perception, emotion and memory as well as advanced motor function.